{
  "gene_symbol": "MSRB1",
  "gene_name": "Methionine-R-sulfoxide reductase B1",
  "term_label": "nucleus",
  "gene": "UniProtKB:Q9NZV6",
  "term_id": "GO:0005634"
}